{
  "term_id": "GO:0004896",
  "gene": "UniProtKB:Q8N6P7",
  "gene_name": "Interleukin-22 receptor subunit alpha-1",
  "gene_symbol": "IL22RA1",
  "term_label": "cytokine receptor activity"
}